{
  "gene": "UniProtKB:Q9NYW8",
  "gene_name": "RB-associated KRAB zinc finger protein",
  "term_label": "RNA polymerase II cis-regulatory region sequence-specific DNA binding",
  "term_id": "GO:0000978",
  "gene_symbol": "RBAK"
}